{
  "term_label": "type I interferon-mediated signaling pathway",
  "gene_name": "Interferon alpha-21",
  "term_id": "GO:0060337",
  "gene": "UniProtKB:P01568",
  "gene_symbol": "IFNA21"
}